positive regulation of T-helper cell differentiation [GO:0045624] (biological process) Definition: Any process that activates or increases the frequency, rate or extent of T-helper cell differentiation. Also known as: up regulation of T-helper cell differentiation, up-regulation of T-helper cell differentiation, upregulation of T-helper cell differentiation, activation of T-helper cell differentiation, stimulation of T-helper cell differentiation, positive regulation of T-helper cell development Note: Note that immunologists typically use the word 'development' to refer to cells of B or T cell lineages undergoing the process that GO describes as 'cell differentiation'. Relationships: is_a positive regulation of immune effector process [GO:0002699]; is a type of positive regulation of CD4-positive, alpha-beta T cell differentiation [GO:0043372]; is_a regulation of T-helper cell differentiation [GO:0045622]; is a type of positive regulation of immune response [GO:0050778]; positively regulates T-helper cell differentiation [GO:0042093] Subtypes: positive regulation of T-helper 1 cell differentiation [GO:0045627], positive regulation of T-helper 2 cell differentiation [GO:0045630], GO:2000321 Sources: GOC:go_curators